{
  "term_id": "GO:0008431",
  "gene_symbol": "AFM",
  "gene": "UniProtKB:P43652",
  "gene_name": "Afamin",
  "term_label": "vitamin E binding"
}